germ-line cyst formation [GO:0048134] (biological process) Relationships: is a type of GO:0008283; is part of germ cell development [GO:0007281] References: PMID:10370240, PMID:21681920 Sources: GOC:jid Subtypes: GO:0048135, male germ-line cyst formation [GO:0048136] Definition: Formation of a group of interconnected cells derived from a single gonial founder cell. Also known as: germline cyst formation